PUMA-BCL-xl complex [GO:0097143] (cellular component) Definition: A heterodimeric protein complex consisting of PUMA and BCL-xl, members of the Bcl-2 family of anti- and proapoptotic regulators. References: PMID:14634621 Sources: GOC:so Relationships: is a type of Bcl-2 family protein complex [GO:0097136]